dense core granule biogenesis [GO:0061110] (biological process) Definition: A cellular process that results in the biosynthesis of constituent macromolecules, assembly, and arrangement of constituent parts of a dense core granule. Includes biosynthesis of constituent macromolecules, and those macromolecular modifications that are involved in synthesis or assembly of the dense core granule. Regulation: regulated by regulation of dense core granule biogenesis [GO:2000705]; negatively regulated by negative regulation of dense core granule biogenesis [GO:2000706]; positively regulated by positive regulation of dense core granule biogenesis [GO:2000707] Sources: GOC:dph Relationships: is a type of GO:0044085